{
  "term_id": "GO:0035725",
  "gene_symbol": "SCNN1D",
  "gene_name": "Amiloride-sensitive sodium channel subunit delta",
  "gene": "UniProtKB:P51172",
  "term_label": "sodium ion transmembrane transport"
}